{
  "gene_symbol": "ZNF629",
  "gene": "UniProtKB:Q9UEG4",
  "term_label": "nucleus",
  "gene_name": "Zinc finger protein 629",
  "term_id": "GO:0005634"
}